{
  "gene": "UniProtKB:Q9NWY4",
  "gene_symbol": "HPF1",
  "gene_name": "Histone PARylation factor 1",
  "term_label": "nucleus",
  "term_id": "GO:0005634"
}